{
  "term_label": "Unknown biological process",
  "gene_symbol": "ZNF826P",
  "term_id": "UNKNOWN:0002",
  "gene_name": "Putative zinc finger protein 826",
  "gene": "UniProtKB:Q6ZT77"
}